{
  "term_label": "Unknown biological process",
  "gene_name": "Uncharacterized protein C9orf50",
  "term_id": "UNKNOWN:0002",
  "gene": "UniProtKB:Q5SZB4",
  "gene_symbol": "C9orf50"
}